{
  "term_id": "GO:0000981",
  "term_label": "DNA-binding transcription factor activity, RNA polymerase II-specific",
  "gene_symbol": "FOXJ2",
  "gene": "UniProtKB:Q9P0K8",
  "gene_name": "Forkhead box protein J2"
}